hexose-phosphate:phosphate antiporter activity [GO:0015526] (molecular function) Definition: Enables the transfer of a solute or solutes from one side of a membrane to the other according to the reaction: hexose phosphate(out) + phosphate(in) = hexose phosphate(in) +  phosphate(out). Sources: TC:2.A.1.4.1 Subtypes: glucose 6-phosphate:phosphate antiporter activity [GO:0061513] Relationships: is a type of hexose phosphate transmembrane transporter activity [GO:0015119]; is a type of organophosphate:phosphate antiporter activity [GO:0015315] Also known as: hexose-phosphate:inorganic phosphate antiporter activity